{
  "term_label": "extracellular space",
  "gene_symbol": "IFNL3",
  "term_id": "GO:0005615",
  "gene_name": "Interferon lambda-3",
  "gene": "UniProtKB:Q8IZI9"
}